pH elevation [GO:0045852] (biological process) Definition: Any process that increases the internal pH of an organism, part of an organism or a cell, measured by the concentration of the hydrogen ion. Relationships: is a type of regulation of pH [GO:0006885] Sources: GOC:go_curators